{
  "term_id": "GO:0007165",
  "term_label": "signal transduction",
  "gene_name": "14-3-3 protein theta",
  "gene": "UniProtKB:P27348",
  "gene_symbol": "YWHAQ"
}